{
  "gene_name": "Selenocysteine insertion sequence-binding protein 2",
  "term_id": "GO:0005739",
  "gene_symbol": "SECISBP2",
  "term_label": "mitochondrion",
  "gene": "UniProtKB:Q96T21"
}